{
  "term_id": "GO:0005739",
  "gene": "UniProtKB:Q15526",
  "gene_symbol": "SURF1",
  "term_label": "mitochondrion",
  "gene_name": "Surfeit locus protein 1"
}